pyrimidine nucleoside binding [GO:0001884] (molecular function) Relationships: is_a GO:0001882 Definition: Binding to a pyrimidine nucleoside, a compound consisting of a pyrimidine base linked either to ribose or deoxyribose. Subtypes: GO:0032548, pyrimidine ribonucleoside binding [GO:0032551] Sources: GOC:hjd